{
  "gene_name": "Solute carrier family 35 member G1",
  "term_id": "UNKNOWN:0001",
  "term_label": "Unknown molecular function",
  "gene": "UniProtKB:Q2M3R5",
  "gene_symbol": "SLC35G1"
}